ascospore-type prospore-specific spindle pole body remodeling [GO:0031322] (BP) Also known as: ascospore-type prospore-specific spindle pole body remodelling, forespore specific spindle pole body remodeling, forespore-specific spindle pole body remodeling, prospore-specific spindle pole body remodeling, sporulation-specific spindle pole body remodeling, ascospore-type prospore-specific spindle pole body modification Definition: A spindle pole body (SPB) organization process that takes place during the second meiotic division during ascospore formation and results in the structural reorganization of the SPB; includes the recruitment of sporulation-specific proteins to the outer plaque to form the meiotic outer plaque (MOP). References: PMID:14702385 Sources: GOC:mah Relationships: is a type of GO:1903046; is part of microtubule cytoskeleton organization [GO:0000226]; is part of GO:0031321